{
  "gene_symbol": "MYO16",
  "term_label": "nucleoplasm",
  "term_id": "GO:0005654",
  "gene": "UniProtKB:Q9Y6X6",
  "gene_name": "Unconventional myosin-XVI"
}